{
  "term_id": "GO:0005929",
  "term_label": "cilium",
  "gene_name": "Tubby-related protein 2",
  "gene_symbol": "TULP2",
  "gene": "UniProtKB:O00295"
}